positive regulation of hematopoietic stem cell proliferation [GO:1902035] (biological process) Definition: Any process that activates or increases the frequency, rate or extent of hematopoietic stem cell proliferation. References: PMID:23403623 Sources: GOC:TermGenie Also known as: positive regulation of hemopoietic stem cell proliferation, up regulation of hematopoietic stem cell proliferation, up regulation of hemopoietic stem cell proliferation, up-regulation of hematopoietic stem cell proliferation, up-regulation of hemopoietic stem cell proliferation, upregulation of hematopoietic stem cell proliferation, upregulation of hemopoietic stem cell proliferation, activation of hematopoietic stem cell proliferation, activation of hemopoietic stem cell proliferation Relationships: is a type of GO:1902033; is a type of positive regulation of stem cell proliferation [GO:2000648]; positively regulates hematopoietic stem cell proliferation [GO:0071425]